{
  "gene_symbol": "LAMB3",
  "gene": "UniProtKB:Q13751",
  "term_id": "GO:0005201",
  "gene_name": "Laminin subunit beta-3",
  "term_label": "extracellular matrix structural constituent"
}